regulation of mRNA modification [GO:0090365] (biological process) Subtypes: positive regulation of mRNA modification [GO:0090366], negative regulation of mRNA modification [GO:0090367] References: PMID:14559896 Sources: GOC:dph, GOC:sl, GOC:tb Also known as: regulation of mRNA editing Relationships: is a type of regulation of mRNA metabolic process [GO:1903311]; regulates GO:0016556 Definition: Any process that modulates the rate, frequency, or extent of the covalent alteration of one or more nucleotides within an mRNA molecule to produce an mRNA molecule with a sequence that differs from that coded genetically.